glycine betaine:sodium:chloride symporter activity [GO:0140814] (molecular function) Also known as: sodium/chloride-dependent glycine betaine transporter activity References: PMID:10358010 Relationships: is a type of GO:0015199; is a type of sodium:chloride symporter activity [GO:0015378]; is part of glycine betaine transport [GO:0031460] Definition: Enables the transfer of a solute or solutes from one side of a membrane to the other according to the reaction: glycine betaine(out) + Na+(out) + Cl-(out)= glycine betaine(in) + Na+(in) + Cl-(in).